{
  "term_id": "GO:0005737",
  "gene_symbol": "SULT1C4",
  "term_label": "cytoplasm",
  "gene": "UniProtKB:O75897",
  "gene_name": "Sulfotransferase 1C4"
}